{
  "term_id": "UNKNOWN:0002",
  "gene": "UniProtKB:Q8WXA9",
  "gene_name": "Splicing regulatory glutamine_lysine-rich protein 1",
  "term_label": "Unknown biological process",
  "gene_symbol": "SREK1"
}